{
  "term_label": "negative regulation of TORC1 signaling",
  "gene_name": "Ataxin-3-like protein",
  "term_id": "GO:1904262",
  "gene": "UniProtKB:Q9H3M9",
  "gene_symbol": "ATXN3L"
}